{
  "term_label": "phosphatidylinositol 3-kinase/protein kinase B signal transduction",
  "gene_symbol": "PIK3C2A",
  "gene_name": "Phosphatidylinositol 4-phosphate 3-kinase C2 domain-containing subunit alpha",
  "term_id": "GO:0043491",
  "gene": "UniProtKB:O00443"
}